{
  "gene": "UniProtKB:Q9UKT7",
  "gene_name": "F-box_LRR-repeat protein 3",
  "term_label": "Unknown molecular function",
  "gene_symbol": "FBXL3",
  "term_id": "UNKNOWN:0001"
}